{
  "gene_symbol": "GLRA1",
  "gene": "UniProtKB:P23415",
  "term_id": "GO:1902476",
  "term_label": "chloride transmembrane transport",
  "gene_name": "Glycine receptor subunit alpha-1"
}